{
  "gene_symbol": "CD164",
  "term_label": "lysosome",
  "gene": "UniProtKB:Q04900",
  "gene_name": "Sialomucin core protein 24",
  "term_id": "GO:0005764"
}